{
  "term_id": "GO:0005739",
  "term_label": "mitochondrion",
  "gene": "UniProtKB:Q9NQH7",
  "gene_symbol": "XPNPEP3",
  "gene_name": "Xaa-Pro aminopeptidase 3"
}